{
  "term_id": "GO:0016787",
  "term_label": "hydrolase activity",
  "gene_name": "Lysoplasmalogenase-like protein TMEM86A",
  "gene_symbol": "TMEM86A",
  "gene": "UniProtKB:Q8N2M4"
}